{
  "term_label": "plasma membrane",
  "term_id": "GO:0005886",
  "gene_name": "Lysophosphatidic acid receptor 2",
  "gene": "UniProtKB:Q9HBW0",
  "gene_symbol": "LPAR2"
}